{
  "gene_name": "Germ cell nuclear acidic protein",
  "gene": "UniProtKB:Q96QF7",
  "term_label": "Unknown biological process",
  "term_id": "UNKNOWN:0002",
  "gene_symbol": "GCNA"
}